{
  "gene_symbol": "TCP10L",
  "term_id": "UNKNOWN:0001",
  "gene_name": "T-complex protein 10A homolog 1",
  "term_label": "Unknown molecular function",
  "gene": "UniProtKB:Q8TDR4"
}